{
  "gene": "UniProtKB:P81172",
  "gene_name": "Hepcidin",
  "term_label": "negative regulation of iron ion transmembrane transport",
  "term_id": "GO:0034760",
  "gene_symbol": "HAMP"
}